{
  "gene_symbol": "MTRNR2L5",
  "gene_name": "Humanin-like 5",
  "term_id": "GO:0048019",
  "term_label": "receptor antagonist activity",
  "gene": "UniProtKB:P0CJ72"
}